intracellular anatomical structure [GO:0005622] (cellular component) Definition: A component of a cell contained within (but not including) the plasma membrane. In eukaryotes it includes the nucleus and cytoplasm. Sources: ISBN:0198506732 Also known as: internal to cell, intracellular, protoplasm, nucleocytoplasm, protoplast Relationships: is a type of cellular anatomical structure [GO:0110165] Subtypes: GO:0005727, GO:0016234, GO:0044100, extrachromosomal DNA [GO:0046821], metaphase plate [GO:0070090], GO:0070477